{
  "gene_symbol": "TMEM164",
  "term_label": "Unknown molecular function",
  "term_id": "UNKNOWN:0001",
  "gene_name": "Transmembrane protein 164",
  "gene": "UniProtKB:Q5U3C3"
}